{
  "gene_name": "ADP_ATP translocase 4",
  "term_id": "GO:0005757",
  "gene_symbol": "SLC25A31",
  "term_label": "mitochondrial permeability transition pore complex",
  "gene": "UniProtKB:Q9H0C2"
}